{
  "term_id": "UNKNOWN:0002",
  "term_label": "Unknown biological process",
  "gene": "UniProtKB:Q96LP2",
  "gene_symbol": "FAM81B",
  "gene_name": "Protein FAM81B"
}